{
  "term_id": "GO:0051082",
  "term_label": "unfolded protein binding",
  "gene_symbol": "GRPEL2",
  "gene_name": "GrpE protein homolog 2, mitochondrial",
  "gene": "UniProtKB:Q8TAA5"
}